{
  "term_label": "plasma membrane",
  "gene_symbol": "GPRC5D",
  "term_id": "GO:0005886",
  "gene_name": "G-protein coupled receptor family C group 5 member D",
  "gene": "UniProtKB:Q9NZD1"
}